{
  "gene_name": "S-methylmethionine--homocysteine S-methyltransferase BHMT2",
  "term_id": "GO:0071267",
  "gene": "UniProtKB:Q9H2M3",
  "term_label": "L-methionine salvage",
  "gene_symbol": "BHMT2"
}